{
  "gene": "UniProtKB:Q96K76",
  "gene_name": "Ubiquitin carboxyl-terminal hydrolase 47",
  "gene_symbol": "USP47",
  "term_label": "cytosol",
  "term_id": "GO:0005829"
}